regulation of axon extension involved in axon guidance [GO:0048841] (biological process) Relationships: is a type of regulation of axon extension [GO:0030516]; regulates axon extension involved in axon guidance [GO:0048846] Subtypes: positive regulation of axon extension involved in axon guidance [GO:0048842], negative regulation of axon extension involved in axon guidance [GO:0048843] Definition: Any process that modulates the frequency, rate or extent of axon extension involved in axon guidance. Sources: GOC:devbiol